{
  "gene_symbol": "PLAAT4",
  "gene": "UniProtKB:Q9UL19",
  "gene_name": "Phospholipase A and acyltransferase 4",
  "term_label": "N-acyltransferase activity",
  "term_id": "GO:0016410"
}